{
  "gene_name": "Tyrosine-protein phosphatase non-receptor type 13",
  "gene_symbol": "PTPN13",
  "term_id": "GO:0005634",
  "term_label": "nucleus",
  "gene": "UniProtKB:Q12923"
}